nickel cation transmembrane transport [GO:0035444] (biological process) Definition: The directed movement of nickel (Ni) cations across a membrane by means of some agent such as a transporter or pore. Subtypes: nickel cation import across plasma membrane [GO:0098716] Relationships: is a type of nickel cation transport [GO:0015675]; is a type of monoatomic cation transmembrane transport [GO:0098655] Sources: GOC:vw Note: Note that this term is not intended for use in annotating lateral movement within membranes. Also known as: nickel cation membrane transport